nitrobenzene biosynthetic process [GO:1900999] (biological process) Definition: The chemical reactions and pathways resulting in the formation of nitrobenzene. Sources: GOC:TermGenie, GOC:yaf, UniPathway:UPA00923 Relationships: is a type of biosynthetic process [GO:0009058]; is a type of nitrobenzene metabolic process [GO:0018916] Also known as: nitrobenzene anabolism, nitrobenzene biosynthesis, nitrobenzene formation, nitrobenzene synthesis